{
  "gene_symbol": "HYAL2",
  "term_label": "hyaluronoglucuronidase activity",
  "gene": "UniProtKB:Q12891",
  "gene_name": "Hyaluronidase-2",
  "term_id": "GO:0033906"
}